{
  "gene_symbol": "OR4D10",
  "term_id": "GO:0005886",
  "gene_name": "Olfactory receptor 4D10",
  "gene": "UniProtKB:Q8NGI6",
  "term_label": "plasma membrane"
}